{
  "term_id": "GO:0000727",
  "term_label": "double-strand break repair via break-induced replication",
  "gene_symbol": "MCM3",
  "gene_name": "DNA replication licensing factor MCM3",
  "gene": "UniProtKB:P25205"
}